{
  "gene_name": "Immunoglobulin kappa joining 1",
  "term_label": "Unknown molecular function",
  "gene_symbol": "IGKJ1",
  "term_id": "UNKNOWN:0001",
  "gene": "UniProtKB:A0A0A0MT89"
}